{
  "term_label": "adenylate cyclase-activating G protein-coupled receptor signaling pathway",
  "gene": "UniProtKB:P10644",
  "gene_symbol": "PRKAR1A",
  "gene_name": "cAMP-dependent protein kinase type I-alpha regulatory subunit",
  "term_id": "GO:0007189"
}